{
  "gene": "UniProtKB:Q643R3",
  "term_label": "lysophosphatidic acid acyltransferase activity",
  "gene_symbol": "LPCAT4",
  "gene_name": "Lysophospholipid acyltransferase LPCAT4",
  "term_id": "GO:0042171"
}